{
  "gene_symbol": "COL25A1",
  "gene": "UniProtKB:Q9BXS0",
  "term_id": "UNKNOWN:0003",
  "term_label": "Unknown cellular component",
  "gene_name": "Collagen alpha-1(XXV) chain"
}